{
  "gene_name": "FERM domain-containing protein 4B",
  "gene_symbol": "FRMD4B",
  "term_id": "GO:0005912",
  "gene": "UniProtKB:Q9Y2L6",
  "term_label": "adherens junction"
}